interleukin-4 receptor complex [GO:0016516] (cellular component) Also known as: IL-4 receptor complex Relationships: is_a plasma membrane signaling receptor complex [GO:0098802] References: PMID:10358772 Definition: A protein complex that binds interleukin-4 (IL-4) and consists of an alpha chain that binds IL-4 with high affinity and a gamma common chain that also forms part of the interleukin-2 receptor.